{
  "gene_name": "Tumor necrosis factor ligand superfamily member 18",
  "gene": "UniProtKB:Q9UNG2",
  "term_label": "tumor necrosis factor receptor superfamily binding",
  "term_id": "GO:0032813",
  "gene_symbol": "TNFSF18"
}